positive regulation of small intestinal transit [GO:0120058] (biological process) Definition: Any process that increases the frequency, rate or extent of any small intestinal transit process, the migration of ingested material along the length of the small intestine. References: PMID:15890336 Sources: GOC:sl Also known as: positive regulation of small bowel transit, positive regulation of small intestine transit Relationships: is a type of GO:0060456; is a type of regulation of small intestinal transit [GO:0120057]; positively regulates small intestinal transit [GO:0120055]